positive regulation of pyrimidine-containing compound salvage [GO:1903931] (biological process) References: PMID:23695302 Sources: GOC:TermGenie, GO_REF:0000058 Also known as: up regulation of pyrimidine-containing compound salvage, up-regulation of pyrimidine-containing compound salvage, upregulation of pyrimidine-containing compound salvage, activation of pyrimidine-containing compound salvage, activation of pyrimidine salvage, positive regulation of pyrimidine salvage, up regulation of pyrimidine salvage, up-regulation of pyrimidine salvage, upregulation of pyrimidine salvage Definition: Any process that activates or increases the frequency, rate or extent of pyrimidine-containing compound salvage. Relationships: is a type of positive regulation of biosynthetic process [GO:0009891]; is a type of GO:1903930; positively regulates GO:0008655